{
  "gene_name": "Olfactory receptor 10S1",
  "term_id": "GO:0005886",
  "term_label": "plasma membrane",
  "gene": "UniProtKB:Q8NGN2",
  "gene_symbol": "OR10S1"
}